{
  "gene_name": "ATP-binding cassette sub-family G member 8",
  "gene_symbol": "ABCG8",
  "term_id": "GO:0055085",
  "term_label": "transmembrane transport",
  "gene": "UniProtKB:Q9H221"
}